{
  "term_label": "microtubule cytoskeleton organization",
  "gene_symbol": "TUBB4B",
  "term_id": "GO:0000226",
  "gene_name": "Tubulin beta-4B chain",
  "gene": "UniProtKB:P68371"
}